{
  "gene_name": "Dolichyl-diphosphooligosaccharide--protein glycosyltransferase subunit 4",
  "term_id": "UNKNOWN:0001",
  "gene": "UniProtKB:P0C6T2",
  "gene_symbol": "OST4",
  "term_label": "Unknown molecular function"
}